regulation of leukocyte proliferation [GO:0070663] (biological process) Definition: Any process that modulates the frequency, rate or extent of leukocyte proliferation. Subtypes: regulation of mononuclear cell proliferation [GO:0032944], negative regulation of leukocyte proliferation [GO:0070664], positive regulation of leukocyte proliferation [GO:0070665], regulation of mast cell proliferation [GO:0070666], GO:0090289, regulation of macrophage proliferation [GO:0120040] Relationships: is a type of GO:0042127; regulates leukocyte proliferation [GO:0070661] Sources: GOC:add, GOC:mah